vascular associated smooth muscle cell proliferation [GO:1990874] (biological process) Regulation: regulated by GO:1904705; negatively regulated by negative regulation of vascular associated smooth muscle cell proliferation [GO:1904706]; positively regulated by positive regulation of vascular associated smooth muscle cell proliferation [GO:1904707] Also known as: VSMC proliferation, vascular smooth muscle cell proliferation Relationships: is a type of smooth muscle cell proliferation [GO:0048659] Definition: The multiplication or reproduction of vascular smooth muscle cells, resulting in the expansion of a cell population. A vascular smooth muscle cell is a non-striated, elongated, spindle-shaped cell found lining the blood vessels. References: PMID:23246467